eyespot apparatus [GO:1990413] (cellular component) Also known as: eyespot, stigma Definition: A small pigmented organelle used in single-celled organisms to detect light. Sources: Wikipedia:Eyespot_apparatus Relationships: is a type of intracellular membrane-bounded organelle [GO:0043231]